{
  "term_label": "mitochondrion",
  "gene": "UniProtKB:P42126",
  "term_id": "GO:0005739",
  "gene_symbol": "ECI1",
  "gene_name": "Enoyl-CoA delta isomerase 1, mitochondrial"
}